{
  "gene": "UniProtKB:Q0VAK6",
  "term_id": "GO:0005856",
  "gene_symbol": "LMOD3",
  "gene_name": "Leiomodin-3",
  "term_label": "cytoskeleton"
}